prostate epithelial cord arborization involved in prostate glandular acinus morphogenesis [GO:0060527] (biological process) Definition: The branching morphogenesis process in which the prostate epithelial cords branch freely to create the structure of the prostate acini. Relationships: is a type of GO:0060442; is part of prostate glandular acinus morphogenesis [GO:0060526] References: PMID:18977204 Sources: GOC:dph